{
  "gene": "UniProtKB:Q6UWM9",
  "gene_name": "UDP-glucuronosyltransferase 2A3",
  "term_id": "UNKNOWN:0002",
  "gene_symbol": "UGT2A3",
  "term_label": "Unknown biological process"
}